3-dehydrosphinganine reductase activity [GO:0047560] (molecular function) Relationships: is a type of oxidoreductase activity, acting on the CH-OH group of donors, NAD or NADP as acceptor [GO:0016616] Definition: Catalysis of the reaction: NADP+ + sphinganine = 3-dehydrosphinganine + H+ + NADPH. Also known as: 3-ketosphinganine reductase activity, 3-oxosphinganine reductase activity, 3-oxosphinganine:NADPH oxidoreductase activity, D-3-dehydrosphinganine reductase activity, D-3-oxosphinganine reductase activity, D-3-oxosphinganine:B-NADPH oxidoreductase activity, D-erythro-dihydrosphingosine:NADP+ 3-oxidoreductase activity, DSR activity, KTS reductase activity Sources: EC:1.1.1.102, RHEA:22640